salicylaldehyde dehydrogenase (NAD+) activity [GO:0018485] (molecular function) Sources: RHEA:18537 Definition: Catalysis of the reaction: salicylaldehyde + NAD+ + H2O = salicylate + NADH + H+. Also known as: salicylaldehyde:NAD+ oxidoreductase activity Relationships: is a type of GO:0004029